response to microbial phytotoxin [GO:0010188] (biological process) Relationships: is a type of response to toxic substance [GO:0009636] Sources: GOC:sm Definition: Any process that results in a change in state or activity of a cell or an organism (in terms of movement, secretion, enzyme production, gene expression, etc.) as a result of a microbial phytotoxin stimulus. A microbial phytotoxin is a chemical substance produced by microbes which is toxic to plants.